{
  "gene": "UniProtKB:Q8WWR8",
  "gene_name": "Sialidase-4",
  "term_id": "GO:0004308",
  "term_label": "exo-alpha-sialidase activity",
  "gene_symbol": "NEU4"
}